photosynthetic NADP+ reduction [GO:0009780] (biological process) Relationships: is a type of NADPH regeneration [GO:0006740]; is part of photosynthesis, light reaction [GO:0019684] Definition: An NADPH regeneration process that contributes to the light reactions of photosynthesis. The light reactions of photosynthesis use energy from photons to generate high-energy electrons. These electrons are used directly to reduce NADP+ to NADPH. NADPH is a relatively stable molecule and can pass on its hydrogen atom to other molecules in chemical reactions. Sources: GOC:jid, ISBN:0716746840, ISBN:0816017360